{
  "gene": "UniProtKB:Q9NRZ5",
  "gene_symbol": "AGPAT4",
  "term_label": "endomembrane system",
  "term_id": "GO:0012505",
  "gene_name": "1-acyl-sn-glycerol-3-phosphate acyltransferase delta"
}